{
  "gene": "UniProtKB:Q70CQ1",
  "term_label": "Unknown biological process",
  "term_id": "UNKNOWN:0002",
  "gene_symbol": "USP49",
  "gene_name": "Ubiquitin carboxyl-terminal hydrolase 49"
}